{
  "gene_name": "Cytochrome P450 3A43",
  "gene_symbol": "CYP3A43",
  "term_id": "UNKNOWN:0003",
  "gene": "UniProtKB:Q9HB55",
  "term_label": "Unknown cellular component"
}